{
  "term_id": "GO:0005886",
  "gene_name": "Receptor for retinol uptake STRA6",
  "gene_symbol": "STRA6",
  "gene": "UniProtKB:Q9BX79",
  "term_label": "plasma membrane"
}